{
  "gene_symbol": "AGBL1",
  "term_id": "GO:0005737",
  "gene_name": "Cytosolic carboxypeptidase 4",
  "gene": "UniProtKB:Q96MI9",
  "term_label": "cytoplasm"
}